{
  "term_id": "GO:0006629",
  "gene_symbol": "LCAT",
  "term_label": "lipid metabolic process",
  "gene": "UniProtKB:P04180",
  "gene_name": "Phosphatidylcholine-sterol acyltransferase"
}